gamma-aminobutyrate shunt [GO:0006540] (biological process) Note: Note that the third step in this pathway (conversion of succinate semialdehyde to succinate) can be catalyzed by NAD-dependent or NADP-dependent succinate semialdehyde dehydrogenase (EC:1.2.1.24 and EC:1.2.1.79, respectively). Also known as: 4-aminobutyrate shunt, GABA shunt, degradation of glutamate to succinate through GABA, gamma aminobutyrate shunt, glutamate decarboxylation to succinate, glutamate degradation via 4-aminobutyrate, glutamate degradation via GABA Relationships: is a type of succinate metabolic process [GO:0006105]; is a type of L-glutamate catabolic process [GO:0006538]; has part glutamate decarboxylase activity [GO:0004351]; has part 4-aminobutyrate:2-oxoglutarate transaminase activity [GO:0034386] Definition: The chemical reactions and pathways resulting in the formation of succinate from L-glutamate. Also known as GABA (gamma-aminobutyrate) shunt since it channels glutamate into the TCA cycle bypassing two steps of that cycle. There are three enzymes involved in the GABA shunt: glutamate decarboxylase (GAD), GABA aminotransferase (GABA-TA), and succinate semialdehyde dehydrogenase (SSADH). These three enzymes acting in concert to convert glutamate into succinate. The GABA shunt is predominantly associated with neurotransmission in the mammalian brain. It is also present in nonneuronal cells, in plants, in unicellular eukaryotes, and in prokaryotes. References: PMID:12740438